{
  "gene": "UniProtKB:Q13045",
  "gene_name": "Protein flightless-1 homolog",
  "term_label": "myofibril assembly",
  "gene_symbol": "FLII",
  "term_id": "GO:0030239"
}